{
  "gene_name": "Histone deacetylase 1",
  "term_id": "GO:0004407",
  "gene": "UniProtKB:Q13547",
  "term_label": "histone deacetylase activity",
  "gene_symbol": "HDAC1"
}